{
  "gene_symbol": "GREB1L",
  "term_label": "kidney development",
  "gene_name": "GREB1-like protein",
  "term_id": "GO:0001822",
  "gene": "UniProtKB:Q9C091"
}